{
  "gene_name": "Melanotransferrin",
  "term_id": "UNKNOWN:0001",
  "term_label": "Unknown molecular function",
  "gene": "UniProtKB:P08582",
  "gene_symbol": "MELTF"
}